{
  "gene": "UniProtKB:O00451",
  "term_id": "GO:0016167",
  "gene_name": "GDNF family receptor alpha-2",
  "gene_symbol": "GFRA2",
  "term_label": "glial cell-derived neurotrophic factor receptor activity"
}